{
  "gene_name": "Protein FAM90A19",
  "term_label": "Unknown biological process",
  "term_id": "UNKNOWN:0002",
  "gene": "UniProtKB:P0DV76",
  "gene_symbol": "FAM90A19"
}